{
  "gene": "UniProtKB:Q7Z3Z2",
  "term_id": "GO:0060041",
  "gene_name": "Protein RD3",
  "term_label": "retina development in camera-type eye",
  "gene_symbol": "RD3"
}